positive regulation of chemokinesis [GO:1904367] (biological process) Relationships: is a type of positive regulation of response to external stimulus [GO:0032103]; is a type of regulation of chemokinesis [GO:1904365]; positively regulates chemokinesis [GO:0042466] Also known as: up regulation of chemokinesis, up-regulation of chemokinesis, upregulation of chemokinesis, activation of chemokinesis Definition: Any process that activates or increases the frequency, rate or extent of chemokinesis. References: PMID:8679543 Sources: GOC:TermGenie, GO_REF:0000058